codeine catabolic process [GO:2001292] (biological process) Definition: The chemical reactions and pathways resulting in the breakdown of codeine, an alkaloid found in the opium poppy, Papaver somniferum var. album. Codeine has analgesic, anti-tussive and anti-diarrhoeal properties. References: PMID:8845855 Sources: GOC:yaf Relationships: is a type of isoquinoline alkaloid catabolic process [GO:0071274]; is a type of codeine metabolic process [GO:2001291] Also known as: codeine breakdown, codeine catabolism, codeine degradation